{
  "gene_symbol": "SPATA3",
  "gene": "UniProtKB:Q8NHX4",
  "term_label": "Unknown cellular component",
  "term_id": "UNKNOWN:0003",
  "gene_name": "Spermatogenesis-associated protein 3"
}